histone H2B conserved C-terminal lysine deubiquitinase activity [GO:0140935] (molecular function) Definition: A histone deubiquitinase that cleaves ubiquitin from the conserved C-terminal lysine residue of a histone H2B protein to which it is conjugated. The conserved lysine residue is K119 in fission yeast, K123 in budding yeast, and K120 in mammals. Relationships: is a type of GO:0140936 References: PMID:15657442 Also known as: histone conserved C-terminal lysine deubiquitination